{
  "term_id": "GO:0016525",
  "gene_symbol": "THBS2",
  "gene": "UniProtKB:P35442",
  "term_label": "negative regulation of angiogenesis",
  "gene_name": "Thrombospondin-2"
}